{
  "term_label": "extracellular matrix",
  "term_id": "GO:0031012",
  "gene_name": "A disintegrin and metalloproteinase with thrombospondin motifs 19",
  "gene_symbol": "ADAMTS19",
  "gene": "UniProtKB:Q8TE59"
}